actin filament bundle retrograde transport [GO:0061573] (biological process) Definition: A process of actin filament bundle distribution that results in the arrangement of actin filament bundles from the periphery toward the interior of the cell. Relationships: is a type of actin filament bundle distribution [GO:0070650] Sources: GOC:dph Also known as: actin filament cable retrograde transport